{
  "gene_symbol": "DENND2A",
  "term_label": "Unknown molecular function",
  "gene": "UniProtKB:Q9ULE3",
  "gene_name": "DENN domain-containing protein 2A",
  "term_id": "UNKNOWN:0001"
}